{
  "gene": "UniProtKB:Q9NW15",
  "gene_name": "Anoctamin-10",
  "gene_symbol": "ANO10",
  "term_label": "chloride transmembrane transport",
  "term_id": "GO:1902476"
}